{
  "gene_symbol": "ITGAE",
  "term_id": "GO:0098609",
  "term_label": "cell-cell adhesion",
  "gene": "UniProtKB:P38570",
  "gene_name": "Integrin alpha-E"
}